{
  "gene_symbol": "SKA2",
  "gene": "UniProtKB:Q8WVK7",
  "gene_name": "Spindle and kinetochore-associated protein 2",
  "term_id": "GO:0008017",
  "term_label": "microtubule binding"
}